{
  "term_label": "nuclear body",
  "gene": "UniProtKB:Q9BXP5",
  "gene_name": "Serrate RNA effector molecule homolog",
  "gene_symbol": "SRRT",
  "term_id": "GO:0016604"
}